{
  "term_id": "GO:0000298",
  "gene_symbol": "NUDT4B",
  "gene_name": "Diphosphoinositol polyphosphate phosphohydrolase NUDT4B",
  "term_label": "endopolyphosphatase activity",
  "gene": "UniProtKB:A0A024RBG1"
}